{
  "term_label": "Unknown cellular component",
  "gene_name": "Protein FAM236D",
  "gene_symbol": "FAM236D",
  "gene": "UniProtKB:A0A1B0GTK5",
  "term_id": "UNKNOWN:0003"
}